{
  "term_id": "GO:0046887",
  "gene": "UniProtKB:P08949",
  "gene_name": "Neuromedin-B",
  "gene_symbol": "NMB",
  "term_label": "positive regulation of hormone secretion"
}